regulation of neutrophil activation [GO:1902563] (biological process) Definition: Any process that modulates the frequency, rate or extent of neutrophil activation. Relationships: is a type of regulation of leukocyte activation [GO:0002694]; regulates neutrophil activation [GO:0042119] References: PMID:17588661 Sources: GOC:TermGenie Subtypes: GO:1902564, positive regulation of neutrophil activation [GO:1902565]